{
  "gene": "UniProtKB:Q9BQ95",
  "gene_name": "Evolutionarily conserved signaling intermediate in Toll pathway, mitochondrial",
  "gene_symbol": "ECSIT",
  "term_label": "mitochondrion",
  "term_id": "GO:0005739"
}